{
  "gene_name": "Potassium channel subfamily U member 1",
  "term_label": "potassium ion transmembrane transport",
  "term_id": "GO:0071805",
  "gene_symbol": "KCNU1",
  "gene": "UniProtKB:A8MYU2"
}